{
  "gene": "UniProtKB:Q86VQ0",
  "gene_symbol": "LCA5",
  "term_label": "axoneme",
  "term_id": "GO:0005930",
  "gene_name": "Lebercilin"
}